transcription-coupled nucleotide-excision repair, DNA damage recognition [GO:0000716] (biological process) Definition: The identification of lesions on the actively transcribed strand of the DNA duplex as well as a small subset of lesions not recognized by the general nucleotide-excision repair pathway. Relationships: is a type of nucleotide-excision repair, DNA damage recognition [GO:0000715]; is part of transcription-coupled nucleotide-excision repair [GO:0006283] References: PMID:10197977 Sources: GOC:elh Also known as: pyrimidine-dimer repair, DNA damage recognition